glycerol-3-phosphate dehydrogenase (NAD+) activity [GO:0141152] (molecular function) Also known as: L-alpha-glycerol phosphate dehydrogenase activity, L-alpha-glycerophosphate dehydrogenase activity, L-glycerol phosphate dehydrogenase activity, L-glycerophosphate dehydrogenase activity, glycerol 1-phosphate dehydrogenase activity, hydroglycerophosphate dehydrogenase activity, NAD-L-glycerol-3-phosphate dehydrogenase activity, NAD-alpha-glycerophosphate dehydrogenase activity, NAD-dependent glycerol phosphate dehydrogenase activity, NAD-dependent glycerol-3-phosphate dehydrogenase activity, NAD-linked glycerol 3-phosphate dehydrogenase activity, NADH-dihydroxyacetone phosphate reductase activity, alpha-glycerol phosphate dehydrogenase (NAD) activity, alpha-glycerophosphate dehydrogenase (NAD) activity, glycerol phosphate dehydrogenase (NAD) activity, glycerol-3-phosphate dehydrogenase (NAD) activity, glycerol-3-phosphate dehydrogenase [NAD+] activity, glycerophosphate dehydrogenase (NAD) activity Relationships: is a type of glycerol-3-phosphate dehydrogenase [NAD(P)+] activity [GO:0047952] Definition: Catalysis of the reaction: NAD+ + sn-glycerol 3-phosphate = dihydroxyacetone phosphate + H+ + NADH. Sources: RHEA:11092